{
  "term_label": "signaling receptor binding",
  "gene": "UniProtKB:O95406",
  "gene_symbol": "CNIH1",
  "term_id": "GO:0005102",
  "gene_name": "Protein cornichon homolog 1"
}